beta-phosphoglucomutase activity [GO:0008801] (MF) Relationships: is a type of intramolecular phosphotransferase activity [GO:0016868] Sources: EC:5.4.2.6, RHEA:20113 Also known as: beta-D-glucose 1,6-phosphomutase activity Definition: Catalysis of the reaction: beta-D-glucose 1-phosphate = beta-D-glucose 6-phosphate.